{
  "gene_symbol": "TENM4",
  "term_id": "GO:0048666",
  "gene_name": "Teneurin-4",
  "gene": "UniProtKB:Q6N022",
  "term_label": "neuron development"
}